mitochondrial phenylalanyl-tRNA aminoacylation [GO:0070156] (BP) Definition: The process of coupling phenylalanine to phenylalanyl-tRNA in a mitochondrion, catalyzed by phenylalanyl-tRNA synthetase. In tRNA aminoacylation, the amino acid is first activated by linkage to AMP and then transferred to either the 2'- or the 3'-hydroxyl group of the 3'-adenosine residue of the tRNA. Sources: GOC:mah, GOC:mcc Relationships: is a type of phenylalanyl-tRNA aminoacylation [GO:0006432]; is a type of GO:0070127